{
  "term_label": "troponin complex",
  "gene": "UniProtKB:P19429",
  "gene_name": "Troponin I, cardiac muscle",
  "gene_symbol": "TNNI3",
  "term_id": "GO:0005861"
}